{
  "gene_name": "Zinc finger protein 628",
  "gene_symbol": "ZNF628",
  "term_id": "UNKNOWN:0003",
  "gene": "UniProtKB:Q5EBL2",
  "term_label": "Unknown cellular component"
}